{
  "gene_name": "Endomucin",
  "gene_symbol": "EMCN",
  "gene": "UniProtKB:Q9ULC0",
  "term_label": "Unknown biological process",
  "term_id": "UNKNOWN:0002"
}